carotenoid isomerooxygenase activity [GO:0106422] (molecular function) Relationships: is a type of carotenoid dioxygenase activity [GO:0010436] References: PMID:19020100, PMID:19889630 Sources: RHEA:33931 Definition: Catalysis of the reaction: Zeaxanthin + O2 = (3R)-11-cis-3-hydroxyretinal + (3R)-all-trans-3-hydroxyretinal.